response to boron-containing substance [GO:0010036] (BP) Definition: Any process that results in a change in state or activity of a cell or an organism (in terms of movement, secretion, enzyme production, gene expression, etc.) as a result of a boron-containing substance stimulus. Subtypes: GO:0080029 Also known as: response to boron Relationships: is a type of response to chemical [GO:0042221] Sources: GOC:sm